{
  "gene_name": "Tyrosine-protein kinase RYK",
  "gene_symbol": "RYK",
  "gene": "UniProtKB:P34925",
  "term_id": "GO:0010976",
  "term_label": "positive regulation of neuron projection development"
}